{
  "gene_name": "Abl interactor 1",
  "term_label": "SCAR complex",
  "term_id": "GO:0031209",
  "gene_symbol": "ABI1",
  "gene": "UniProtKB:Q8IZP0"
}